{
  "gene": "UniProtKB:P47974",
  "term_label": "mRNA 3'-UTR AU-rich region binding",
  "term_id": "GO:0035925",
  "gene_name": "mRNA decay activator protein ZFP36L2",
  "gene_symbol": "ZFP36L2"
}